{
  "term_label": "Unknown molecular function",
  "term_id": "UNKNOWN:0001",
  "gene_symbol": "FAM149B1",
  "gene_name": "Primary cilium assembly protein FAM149B1",
  "gene": "UniProtKB:Q96BN6"
}